{
  "gene": "UniProtKB:A6NFN9",
  "gene_name": "Protein ANKUB1",
  "gene_symbol": "ANKUB1",
  "term_label": "Unknown cellular component",
  "term_id": "UNKNOWN:0003"
}